{
  "gene": "UniProtKB:Q9UHC3",
  "term_id": "GO:0015280",
  "gene_symbol": "ASIC3",
  "gene_name": "Acid-sensing ion channel 3",
  "term_label": "ligand-gated sodium channel activity"
}